{
  "gene": "UniProtKB:Q6P5S2",
  "gene_symbol": "LEG1",
  "term_id": "UNKNOWN:0002",
  "gene_name": "Protein LEG1 homolog",
  "term_label": "Unknown biological process"
}